{
  "gene_name": "Pleckstrin homology-like domain family A member 3",
  "term_id": "GO:0043065",
  "gene": "UniProtKB:Q9Y5J5",
  "gene_symbol": "PHLDA3",
  "term_label": "positive regulation of apoptotic process"
}